{
  "gene_name": "2-5A-dependent ribonuclease",
  "term_id": "GO:0003723",
  "gene": "UniProtKB:Q05823",
  "gene_symbol": "RNASEL",
  "term_label": "RNA binding"
}